{
  "gene": "UniProtKB:Q6ZVK8",
  "term_id": "UNKNOWN:0002",
  "gene_symbol": "NUDT18",
  "term_label": "Unknown biological process",
  "gene_name": "8-oxo-dGDP phosphatase NUDT18"
}